7S RNA binding [GO:0008312] (molecular function) References: PMID:6181418 Sources: GOC:jl Relationships: is_a RNA binding [GO:0003723] Definition: Binding to a 7S RNA, the RNA component of the signal recognition particle (SRP).